{
  "gene": "UniProtKB:Q92565",
  "term_id": "GO:0032486",
  "term_label": "Rap protein signal transduction",
  "gene_symbol": "RAPGEF5",
  "gene_name": "Rap guanine nucleotide exchange factor 5"
}